tetrahymanol synthase activity [GO:0034073] (molecular function) Note: The reaction occurs in the reverse direction. Also known as: squalene--tetrahymanol cyclase activity, tetrahymanol cyclase activity References: PMID:18033581 Sources: RHEA:30675 Relationships: is_a squalene cyclase activity [GO:0034072] Definition: Catalysis of the reaction: tetrahymanol = squalene + H2O.